Yb body [GO:0070725] (cellular component) Definition: A cytoplasmic part that appears as an electron-dense sphere of around 1.5 micron diameter containing Yb protein found in somatic cells of ovary and testis. There are one to two Yb bodies per cell. Relationships: is a type of cytoplasmic ribonucleoprotein granule [GO:0036464] References: PMID:19433453, PMID:28595904, PMID:31267711 Sources: GOC:sart